{
  "term_id": "UNKNOWN:0001",
  "term_label": "Unknown molecular function",
  "gene": "UniProtKB:A4FU28",
  "gene_symbol": "CTAGE9",
  "gene_name": "cTAGE family member 9"
}